{
  "term_id": "GO:0015141",
  "term_label": "succinate transmembrane transporter activity",
  "gene_symbol": "SLC13A2",
  "gene": "UniProtKB:Q13183",
  "gene_name": "Solute carrier family 13 member 2"
}